negative regulation of germ tube formation [GO:0075012] (biological process) Definition: Any process that stops, prevents, or reduces the frequency, rate or extent of germ tube formation on or near host. The host is defined as the larger of the organisms involved in a symbiotic interaction. Also known as: negative regulation of germ tube formation on or near host Relationships: is a type of negative regulation of developmental process [GO:0051093]; is a type of GO:0075010; negatively regulates germ tube formation [GO:0075009] Sources: GOC:pamgo_curators